{
  "term_id": "UNKNOWN:0003",
  "gene_name": "Putative deoxyribonuclease TATDN3",
  "gene": "UniProtKB:Q17R31",
  "gene_symbol": "TATDN3",
  "term_label": "Unknown cellular component"
}